{
  "term_id": "UNKNOWN:0001",
  "gene_symbol": "MAP7D2",
  "gene": "UniProtKB:Q96T17",
  "gene_name": "MAP7 domain-containing protein 2",
  "term_label": "Unknown molecular function"
}